{
  "term_id": "UNKNOWN:0003",
  "gene_name": "DNA polymerase nu",
  "term_label": "Unknown cellular component",
  "gene": "UniProtKB:Q7Z5Q5",
  "gene_symbol": "POLN"
}